{
  "term_id": "GO:0050911",
  "gene_symbol": "OR2Y1",
  "term_label": "detection of chemical stimulus involved in sensory perception of smell",
  "gene": "UniProtKB:Q8NGV0",
  "gene_name": "Olfactory receptor 2Y1"
}